retinoic acid catabolic process [GO:0034653] (biological process) Relationships: is a type of GO:0016103; is a type of GO:0042363; is a type of retinoic acid metabolic process [GO:0042573]; is a type of monocarboxylic acid catabolic process [GO:0072329] Sources: GOC:BHF, GOC:mah Also known as: retinoic acid breakdown, retinoic acid catabolism, retinoic acid degradation, vitamin A1 acid catabolic process Definition: The chemical reactions and pathways resulting in the breakdown of retinoic acid, one of the three components that makes up vitamin A.